{
  "term_label": "adenosine deaminase activity",
  "term_id": "GO:0004000",
  "gene": "UniProtKB:Q9NZK5",
  "gene_name": "Adenosine deaminase 2",
  "gene_symbol": "ADA2"
}